citronellyl-CoA dehydrogenase activity [GO:0034824] (molecular function) Relationships: is a type of GO:0016628 Definition: Catalysis of the reaction: citronellyl-CoA + NAD+ = cis-geranyl-CoA + NADH + H+. References: PMID:31964529